{
  "gene_symbol": "HRH2",
  "term_label": "dendrite",
  "term_id": "GO:0030425",
  "gene_name": "Histamine H2 receptor",
  "gene": "UniProtKB:P25021"
}